SUMO ligase regulator activity [GO:0180016] (molecular function) References: PMID:19363481, PMID:33446573 Definition: Binds to and modulates the activity of a SUMO ligase. Relationships: is a type of ligase regulator activity [GO:0055103]